(4S)-4-hydroxy-5-phosphonooxypentane-2,3-dione isomerase activity [GO:0002952] (molecular function) Relationships: is a type of intramolecular oxidoreductase activity, interconverting aldoses and ketoses [GO:0016861] Sources: RHEA:44360 Definition: Catalysis of the reaction: (2S)-2-hydroxy-3,4-dioxopentyl phosphate = 3-hydroxy-2,4-dioxopentyl phosphate. Also known as: phospho-AI-2 isomerase activity